{
  "term_label": "regulation of cell migration",
  "gene_name": "Thymosin beta-4",
  "gene": "UniProtKB:P62328",
  "gene_symbol": "TMSB4X",
  "term_id": "GO:0030334"
}